{
  "term_label": "developmental process",
  "gene_name": "Transcription factor 15",
  "term_id": "GO:0032502",
  "gene_symbol": "TCF15",
  "gene": "UniProtKB:Q12870"
}